L-methionine (S)-S-oxide reductase activity [GO:0033744] (MF) Definition: Catalysis of the reaction: [thioredoxin]-disulfide + L-methionine + H2O = L-methionine (S)-S-oxide + [thioredoxin]-dithiol. Sources: RHEA:19993 Also known as: methionine sulfoxide reductase activity, methionine-S-oxide reductase activity, L-methionine-(S)-S-oxide reductase activity, L-methionine:oxidized-thioredoxin S-oxidoreductase activity, L-methionine:thioredoxin-disulfide S-oxidoreductase activity, acetylmethionine sulfoxide reductase activity, fSMsr, free-methionine (S)-S-oxide reductase activity, methyl sulfoxide reductase I and II activity Relationships: is a type of oxidoreductase activity, acting on a sulfur group of donors, disulfide as acceptor [GO:0016671]